{
  "term_label": "plasma membrane",
  "gene_name": "Inactive glutathione hydrolase 2",
  "gene_symbol": "GGT2P",
  "term_id": "GO:0005886",
  "gene": "UniProtKB:P36268"
}